signaling receptor binding [GO:0005102] (molecular function) Sources: GOC:bf, GOC:ceb, ISBN:0198506732 Subtypes: G protein-coupled receptor binding [GO:0001664], GO:0005112, patched binding [GO:0005113], GO:0005115, wishful thinking binding [GO:0005117], sevenless binding [GO:0005118], Toll binding [GO:0005121], torso binding [GO:0005122], scavenger receptor binding [GO:0005124], cytokine receptor binding [GO:0005126], GO:0005158, insulin-like growth factor receptor binding [GO:0005159], ErbB-2 class receptor binding [GO:0005176], integrin binding [GO:0005178], sulfonylurea receptor binding [GO:0017098], aryl hydrocarbon receptor binding [GO:0017162], GO:0030156, semaphorin receptor binding [GO:0030215], intercellular adhesion molecule-3 receptor binding [GO:0030370], GO:0030971, high molecular weight kininogen receptor binding [GO:0030987], acetylcholine receptor binding [GO:0033130], receptor serine/threonine kinase binding [GO:0033612], apolipoprotein receptor binding [GO:0034190], GO:0034987, glutamate receptor binding [GO:0035254], GO:0035325, neuropilin binding [GO:0038191], RIG-I binding [GO:0039552], MDA-5 binding [GO:0039556], neurexin family protein binding [GO:0042043], MHC protein binding [GO:0042287], T cell receptor binding [GO:0042608], CD4 receptor binding [GO:0042609], CD8 receptor binding [GO:0042610], CD70 receptor binding [GO:0042614], CD154 receptor binding [GO:0042615], peroxisome proliferator activated receptor binding [GO:0042975], ErbB-3 class receptor binding [GO:0043125], natural killer cell lectin-like receptor binding [GO:0046703], ephrin receptor binding [GO:0046875], receptor ligand activity [GO:0048018], receptor antagonist activity [GO:0048019], Roundabout binding [GO:0048495], GO:0050786, GABA receptor binding [GO:0050811], GO:0051427, GO:0070325, growth factor receptor binding [GO:0070851], GO:0090722, neuroligin family protein binding [GO:0097109], GO:1990459, GO:1990460, ErbB-4 class receptor binding [GO:1990631], netrin receptor binding [GO:1990890] Also known as: receptor binding, receptor ligand, receptor-associated protein activity Relationships: is a type of GO:0005515 Regulation: regulated by regulation of receptor binding [GO:1900120]; negatively regulated by negative regulation of receptor binding [GO:1900121] Definition: Binding to one or more specific sites on a receptor molecule, a macromolecule that undergoes combination with a hormone, neurotransmitter, drug or intracellular messenger to initiate a change in cell function. Note: Where appropriate, also consider annotating to 'receptor agonist activity ; GO:0048018'.